{
  "gene_symbol": "OR2A4",
  "gene": "UniProtKB:O95047",
  "term_label": "membrane",
  "term_id": "GO:0016020",
  "gene_name": "Olfactory receptor 2A4"
}